quinoprotein glucose dehydrogenase activity [GO:0008876] (molecular function) Also known as: glucose dehydrogenase (pyrroloquinoline-quinone) activity, D-glucose:(pyrroloquinoline-quinone) 1-oxidoreductase activity, D-glucose:ubiquinone oxidoreductase activity, glucose dehydrogenase (PQQ-dependent) activity, quinoprotein D-glucose dehydrogenase activity Sources: RHEA:22152 Relationships: is a type of glucose dehydrogenase activity [GO:0004344]; is a type of oxidoreductase activity, acting on the CH-OH group of donors, quinone or similar compound as acceptor [GO:0016901] Definition: Catalysis of the reaction: D-glucose + ubiquinone = D-glucono-1,5-lactone + ubiquinol.